N4-(beta-N-acetylglucosaminyl)-L-asparaginase activity [GO:0003948] (molecular function) Sources: EC:3.5.1.26, RHEA:11544 Also known as: 4-N-(beta-N-acetyl-D-glucosaminyl)-L-asparagine amidohydrolase activity, N-aspartyl-beta-glucosaminidase activity, N4-(beta-N-acetyl-D-glucosaminyl)-L-asparagine amidohydrolase activity, aspartylglucosaminidase activity, aspartylglucosylaminase activity, aspartylglucosylamine deaspartylase activity, aspartylglucosylaminidase activity, aspartylglycosylamine amidohydrolase activity, beta-aspartylglucosylamine amidohydrolase activity, glucosylamidase activity, glycosylasparaginase activity Relationships: is a type of hydrolase activity, acting on carbon-nitrogen (but not peptide) bonds, in linear amides [GO:0016811] Definition: Catalysis of the reaction: N(4)-(beta-N-acetyl-D-glucosaminyl)-L-asparagine + H2O = N-acetyl-beta-D-glucosaminylamine + L-aspartate + H+.